{
  "gene_name": "A-kinase anchor protein inhibitor 1",
  "term_label": "Unknown cellular component",
  "gene_symbol": "AKAIN1",
  "term_id": "UNKNOWN:0003",
  "gene": "UniProtKB:P0CW23"
}